{
  "term_label": "chemokine-mediated signaling pathway",
  "gene_name": "C-C motif chemokine 18",
  "gene": "UniProtKB:P55774",
  "gene_symbol": "CCL18",
  "term_id": "GO:0070098"
}